{
  "gene": "UniProtKB:Q8NBR6",
  "gene_symbol": "MINDY2",
  "gene_name": "Ubiquitin carboxyl-terminal hydrolase MINDY-2",
  "term_id": "GO:0005654",
  "term_label": "nucleoplasm"
}